{
  "gene_symbol": "GRAPL",
  "gene_name": "GRB2-related adapter protein-like",
  "term_id": "GO:0030971",
  "term_label": "receptor tyrosine kinase binding",
  "gene": "UniProtKB:Q8TC17"
}